ascospore-type prospore [GO:0042764] (cellular component) Definition: An immature spore undergoing development. The spore usually consists of nucleic acid, prospore membrane(s) that encase the nucleic acid, and ultimately a cell wall that covers the membrane(s). This type of spore is observed in ascospore-forming fungi. Relationships: is a type of intracellular immature spore [GO:0042763] Sources: GOC:go_curators